negative regulation of mitotic recombination-dependent replication fork processing [GO:0120291] (biological process) Definition: Any process that inhibits or decreases the rate of mitotic recombination-dependent replication fork processing. Suppression of recombination at replication forks is necessary to prevent template switching. Relationships: is a type of negative regulation of cell cycle process [GO:0010948]; is a type of GO:0051053; is a type of regulation of mitotic recombination-dependent replication fork processing [GO:1903221]; negatively regulates mitotic recombination-dependent replication fork processing [GO:1990426] Also known as: maintenance of template fidelity during replication fork processing, negative regulation of template switch recombination involved in replication fork processing, suppression of template switching during replication fork processing, negative regulation of mitotic recombination involved in replication fork processing References: PMID:28586299, PMID:30667359, PMID:31149897 Sources: GOC:krc, GOC:mah